{
  "term_label": "Unknown cellular component",
  "gene": "UniProtKB:Q3LHN2",
  "term_id": "UNKNOWN:0003",
  "gene_symbol": "KRTAP19-2",
  "gene_name": "Keratin-associated protein 19-2"
}